proton channel activity [GO:0015252] (molecular function) Also known as: hydrogen ion channel activity Subtypes: voltage-gated proton channel activity [GO:0030171], proton-transporting ATP synthase activity, rotational mechanism [GO:0046933] Sources: GOC:mtg_transport, GOC:pr, ISBN:0815340729 Definition: Enables the facilitated diffusion of a hydrogen ion (by an energy-independent process) involving passage through a transmembrane aqueous pore or channel without evidence for a carrier-mediated mechanism. Relationships: is a type of monoatomic cation channel activity [GO:0005261]; is a type of proton transmembrane transporter activity [GO:0015078]